{
  "term_id": "GO:0008375",
  "gene_name": "Alpha-1,4-N-acetylglucosaminyltransferase",
  "gene": "UniProtKB:Q9UNA3",
  "term_label": "acetylglucosaminyltransferase activity",
  "gene_symbol": "A4GNT"
}